{
  "term_id": "GO:0009755",
  "gene": "UniProtKB:Q8WXD0",
  "gene_symbol": "RXFP2",
  "gene_name": "Relaxin receptor 2",
  "term_label": "hormone-mediated signaling pathway"
}